convergent extension involved in notochord morphogenesis [GO:1904126] (biological process) References: PMID:24892953 Sources: GOC:TermGenie, GOC:dph, GO_REF:0000060 Relationships: is a type of convergent extension involved in gastrulation [GO:0060027]; is a type of GO:0060029; is part of notochord morphogenesis [GO:0048570] Definition: Any convergent extension that is involved in notochord morphogenesis. Regulation: regulated by GO:1904136; negatively regulated by negative regulation of convergent extension involved in notochord morphogenesis [GO:1904137]; positively regulated by positive regulation of convergent extension involved in notochord morphogenesis [GO:1904138]